T-helper 2 cell activation [GO:0035712] (biological process) Relationships: is a type of CD4-positive, alpha-beta T cell activation [GO:0035710] Also known as: Th2 cell activation Definition: The change in morphology and behavior of a T helper 2 cell resulting from exposure to a mitogen, cytokine, chemokine, cellular ligand, or an antigen for which it is specific. Regulation: regulated by GO:2000569; positively regulated by positive regulation of T-helper 2 cell activation [GO:2000570] Sources: CL:0000546, GOC:BHF